{
  "gene": "UniProtKB:P16333",
  "term_id": "GO:0036493",
  "gene_symbol": "NCK1",
  "gene_name": "Cytoplasmic protein NCK1",
  "term_label": "positive regulation of translation in response to endoplasmic reticulum stress"
}